{
  "gene_name": "Tripartite motif-containing protein 59",
  "gene_symbol": "TRIM59",
  "term_id": "UNKNOWN:0003",
  "gene": "UniProtKB:Q8IWR1",
  "term_label": "Unknown cellular component"
}